carboxysome [GO:0031470] (CC) Definition: An organelle consisting of a proteinaceous coat and enzymes for the fixation of CO2. It augments the concentration of CO2 in the vicinity of RuBisCO to increase the efficiency of CO2 fixation under atmospheric conditions. Relationships: is a type of bacterial microcompartment [GO:0031469] References: PMID:28934381, PMID:8157606, PMID:8491708 Sources: GOC:js